{
  "term_label": "plasma membrane",
  "term_id": "GO:0005886",
  "gene": "UniProtKB:O00254",
  "gene_symbol": "F2RL2",
  "gene_name": "Proteinase-activated receptor 3"
}